beta-amyrin 16beta-monooxygenase activity [GO:0102601] (MF) Definition: Catalysis of the reaction: beta-amyrin + O2 + reduced [NADPH--hemoprotein reductase] = H+ + H2O + maniladiol + oxidized [NADPH--hemoprotein reductase]. Sources: EC:1.14.14.63 Also known as: cytochrome P450 dependent beta-amyrin 16beta-hydroxylase activity Relationships: is a type of oxidoreductase activity, acting on paired donors, with incorporation or reduction of molecular oxygen, reduced flavin or flavoprotein as one donor, and incorporation of one atom of oxygen [GO:0016712]